glucosylceramide catabolic process [GO:0006680] (biological process) Also known as: glucosylceramide breakdown, glucosylceramide catabolism, glucosylceramide degradation Definition: The chemical reactions and pathways resulting in the breakdown of glucosylceramides, any compound formed by the replacement of the glycosidic hydroxyl group of a cyclic form of glucose by a ceramide group. Regulation: regulated by regulation of glucosylceramide catabolic process [GO:2000752]; positively regulated by positive regulation of glucosylceramide catabolic process [GO:2000753] Sources: GOC:ai Relationships: is a type of glucosylceramide metabolic process [GO:0006678]; is_a glycosylceramide catabolic process [GO:0046477]